{
  "term_id": "GO:0030301",
  "gene_symbol": "APOB",
  "gene_name": "Apolipoprotein B-100",
  "term_label": "cholesterol transport",
  "gene": "UniProtKB:P04114"
}